glycosaminoglycan biosynthetic process [GO:0006024] (biological process) Subtypes: peptidoglycan biosynthetic process [GO:0009252], GO:0030213 Relationships: is a type of aminoglycan biosynthetic process [GO:0006023]; is a type of GO:0030203 Also known as: glycosaminoglycan anabolism, glycosaminoglycan biosynthesis, glycosaminoglycan formation, glycosaminoglycan synthesis Definition: The chemical reactions and pathways resulting in the formation of glycosaminoglycans, any one of a group of linear polysaccharides composed of repeating disaccharide units. References: PMID:38500384